{
  "gene": "UniProtKB:P16112",
  "term_id": "GO:0045202",
  "gene_name": "Aggrecan core protein",
  "term_label": "synapse",
  "gene_symbol": "ACAN"
}